{
  "term_id": "GO:0016020",
  "term_label": "membrane",
  "gene_name": "Bardet-Biedl syndrome 2 protein",
  "gene_symbol": "BBS2",
  "gene": "UniProtKB:Q9BXC9"
}